{
  "gene": "UniProtKB:Q9H336",
  "term_id": "UNKNOWN:0002",
  "gene_name": "Cysteine-rich secretory protein LCCL domain-containing 1",
  "term_label": "Unknown biological process",
  "gene_symbol": "CRISPLD1"
}